negative regulation of protein ADP-ribosylation [GO:0010836] (biological process) Sources: GOC:BHF, GOC:dph, GOC:tb Definition: Any process that decreases the frequency, rate or extent of protein ADP-ribosylation. Protein ADP-ribosylation is the transfer, from NAD, of ADP-ribose to protein amino acids. Relationships: is a type of regulation of protein ADP-ribosylation [GO:0010835]; is a type of negative regulation of catalytic activity [GO:0043086]; negatively regulates GO:1990404 Also known as: negative regulation of protein amino acid ADP-ribosylation